{
  "gene_symbol": "ADAMTS1",
  "gene": "UniProtKB:Q9UHI8",
  "term_id": "GO:0030198",
  "gene_name": "A disintegrin and metalloproteinase with thrombospondin motifs 1",
  "term_label": "extracellular matrix organization"
}